{
  "term_id": "GO:0005768",
  "term_label": "endosome",
  "gene": "UniProtKB:P20337",
  "gene_name": "Ras-related protein Rab-3B",
  "gene_symbol": "RAB3B"
}